negative regulation of toll-like receptor 13 signaling pathway [GO:0034180] (BP) Definition: Any process that stops, prevents, or reduces the frequency, rate, or extent of toll-like receptor 13 signaling pathway. References: PMID:16551253, PMID:17328678 Sources: GOC:add Also known as: negative regulation of TLR13 signaling pathway, negative regulation of toll-like receptor 13 signalling pathway Relationships: is a type of regulation of toll-like receptor 13 signaling pathway [GO:0034179]; is a type of negative regulation of cytoplasmic pattern recognition receptor signaling pathway [GO:0039532]; negatively regulates toll-like receptor 13 signaling pathway [GO:0034178]